{
  "gene": "UniProtKB:Q8TCT8",
  "term_label": "lysosomal membrane",
  "term_id": "GO:0005765",
  "gene_symbol": "SPPL2A",
  "gene_name": "Signal peptide peptidase-like 2A"
}